{
  "term_label": "Unknown cellular component",
  "gene_name": "Interferon-inducible GTPase 5",
  "gene": "UniProtKB:Q6NXR0",
  "gene_symbol": "IRGC",
  "term_id": "UNKNOWN:0003"
}